purine nucleobase transmembrane transporter activity [GO:0005345] (molecular function) Sources: ISBN:0198506732 Subtypes: adenine transmembrane transporter activity [GO:0015207], guanine transmembrane transporter activity [GO:0015208], pyrimidine- and adenosine-specific:sodium symporter activity [GO:0015389], xanthine transmembrane transporter activity [GO:0042907] Also known as: purine base transmembrane transporter activity, purine transmembrane transporter activity Relationships: is a type of GO:0015205; is part of purine nucleobase transmembrane transport [GO:1904823] Definition: Enables the transfer of purine nucleobases, one of the two classes of nitrogen-containing ring compounds found in DNA and RNA, from one side of a membrane to the other.